regulation of promoter clearance from RNA polymerase II promoter [GO:0140845] (biological process) Definition: A process that modulates the frequency, rate or extent of the transition from the initiation to the elongation phases of transcription by RNA polymerase II. References: PMID:28248323 Subtypes: GO:0140846, negative regulation of promoter clearance from RNA polymerase II promoter [GO:0140847] Relationships: is a type of GO:2001141; regulates RNA polymerase II promoter clearance [GO:0001111]